{
  "gene_name": "Cytochrome b-c1 complex subunit 10",
  "gene": "UniProtKB:O14957",
  "term_label": "mitochondrial inner membrane",
  "term_id": "GO:0005743",
  "gene_symbol": "UQCR11"
}